{
  "term_id": "GO:0090575",
  "term_label": "RNA polymerase II transcription regulator complex",
  "gene_name": "Signal transducer and activator of transcription 4",
  "gene": "UniProtKB:Q14765",
  "gene_symbol": "STAT4"
}